{
  "gene": "UniProtKB:P19525",
  "term_label": "regulation of translational initiation",
  "gene_symbol": "EIF2AK2",
  "term_id": "GO:0006446",
  "gene_name": "Interferon-induced, double-stranded RNA-activated protein kinase"
}